{
  "term_id": "UNKNOWN:0002",
  "gene": "UniProtKB:Q13938",
  "gene_name": "Calcyphosin",
  "term_label": "Unknown biological process",
  "gene_symbol": "CAPS"
}